{
  "term_id": "GO:0007422",
  "gene_name": "Adhesion G protein-coupled receptor B2",
  "term_label": "peripheral nervous system development",
  "gene": "UniProtKB:O60241",
  "gene_symbol": "ADGRB2"
}